{
  "term_id": "GO:0046513",
  "gene_symbol": "CERS2",
  "gene_name": "Ceramide synthase 2",
  "gene": "UniProtKB:Q96G23",
  "term_label": "ceramide biosynthetic process"
}